ventricular septum development [GO:0003281] (biological process) Definition: The progression of the ventricular septum over time from its formation to the mature structure. Relationships: is a type of cardiac septum development [GO:0003279]; is part of cardiac ventricle development [GO:0003231] Subtypes: ventricular septum intermedium development [GO:0003282] Also known as: interventricular septum development, septum inferius development Sources: GOC:mtg_heart